positive regulation of bipolar cell growth [GO:0051518] (biological process) Sources: GOC:ai Relationships: is a type of positive regulation of unidimensional cell growth [GO:0051512]; is a type of GO:0051516; RO_0002213 bipolar cell growth [GO:0042815] Subtypes: activation of bipolar cell growth [GO:0051519] Definition: Any process that activates or increases the frequency, rate or extent of bipolar cell growth, polarized growth from both ends of a cell. Also known as: up regulation of bipolar cell growth, up-regulation of bipolar cell growth, upregulation of bipolar cell growth, stimulation of bipolar cell growth